methylenediurea deaminase activity [GO:0047424] (molecular function) Definition: Catalysis of the reaction: 2 H2O + methylenediurea = CO2 + 2 NH3 + N-hydroxymethylurea. Sources: EC:3.5.3.21, MetaCyc:3.5.3.21-RXN, RHEA:15929 Also known as: methylenediurea aminohydrolase activity, methylenediurease activity Relationships: is a type of hydrolase activity, acting on carbon-nitrogen (but not peptide) bonds, in linear amidines [GO:0016813]; is a type of deaminase activity [GO:0019239]